{
  "term_label": "extracellular space",
  "gene": "UniProtKB:P03950",
  "term_id": "GO:0005615",
  "gene_symbol": "ANG",
  "gene_name": "Angiogenin"
}